{
  "gene": "UniProtKB:P0C841",
  "gene_symbol": "FAM66E",
  "term_label": "Unknown cellular component",
  "term_id": "UNKNOWN:0003",
  "gene_name": "Putative protein FAM66E"
}